{
  "gene": "UniProtKB:P06744",
  "term_id": "GO:0048029",
  "gene_symbol": "GPI",
  "term_label": "monosaccharide binding",
  "gene_name": "Glucose-6-phosphate isomerase"
}